{
  "term_id": "GO:0005634",
  "term_label": "nucleus",
  "gene": "UniProtKB:Q9Y5W3",
  "gene_name": "Krueppel-like factor 2",
  "gene_symbol": "KLF2"
}